{
  "gene_name": "Serine_threonine-protein kinase ULK1",
  "gene": "UniProtKB:O75385",
  "gene_symbol": "ULK1",
  "term_id": "GO:0034727",
  "term_label": "piecemeal microautophagy of the nucleus"
}